{
  "term_label": "cytoplasm",
  "term_id": "GO:0005737",
  "gene_symbol": "AKT1S1",
  "gene": "UniProtKB:Q96B36",
  "gene_name": "Proline-rich AKT1 substrate 1"
}